{
  "gene_name": "Large ribosomal subunit protein bL33m",
  "term_label": "Unknown molecular function",
  "gene_symbol": "MRPL33",
  "term_id": "UNKNOWN:0001",
  "gene": "UniProtKB:O75394"
}